{
  "term_id": "UNKNOWN:0001",
  "gene": "UniProtKB:Q6IA17",
  "gene_symbol": "SIGIRR",
  "term_label": "Unknown molecular function",
  "gene_name": "Single Ig IL-1-related receptor"
}